postsynaptic cytosol [GO:0099524] (cellular component) Definition: The region of the cytosol consisting of all cytosol that is part of the postsynapse. Sources: GOC:dos Relationships: is a type of cytosolic region [GO:0099522]; is part of postsynapse [GO:0098794]